{
  "gene": "UniProtKB:P15516",
  "gene_symbol": "HTN3",
  "term_label": "antimicrobial humoral immune response mediated by antimicrobial peptide",
  "gene_name": "Histatin-3",
  "term_id": "GO:0061844"
}